{
  "gene": "UniProtKB:A1L4L8",
  "gene_symbol": "PLAC8L1",
  "gene_name": "PLAC8-like protein 1",
  "term_label": "Unknown molecular function",
  "term_id": "UNKNOWN:0001"
}